DIF-1 biosynthetic process [GO:0031148] (biological process) Also known as: 1-(3,5-dichloro-2,6-dihydroxy-4-methoxyphenyl)hexan-1-one anabolism, 1-(3,5-dichloro-2,6-dihydroxy-4-methoxyphenyl)hexan-1-one biosynthesis, 1-(3,5-dichloro-2,6-dihydroxy-4-methoxyphenyl)hexan-1-one biosynthetic process, 1-(3,5-dichloro-2,6-dihydroxy-4-methoxyphenyl)hexan-1-one formation, 1-(3,5-dichloro-2,6-dihydroxy-4-methoxyphenyl)hexan-1-one synthesis, DIF-1 biosynthesis Relationships: is a type of 1-(3,5-dichloro-2,6-dihydroxy-4-methoxyphenyl)hexan-1-one metabolic process [GO:0031147]; is a type of GO:0042181; is a type of phenol-containing compound biosynthetic process [GO:0046189]; is a type of ether biosynthetic process [GO:1901503] References: PMID:10706822 Sources: GOC:mah Definition: The chemical reactions and pathways resulting in the formation of 1-(3,5-dichloro-2,6-dihydroxy-4-methoxyphenyl)hexan-1-one, also known as DIF-1, differentiation-inducing factor-1. DIF-1 is a secreted chlorinated molecule that controls cell fate during development of Dictyostelium cells.